{
  "gene_symbol": "MYO1D",
  "gene": "UniProtKB:O94832",
  "term_id": "GO:0005737",
  "term_label": "cytoplasm",
  "gene_name": "Unconventional myosin-Id"
}